{
  "gene_symbol": "ERCC6",
  "term_id": "GO:0006283",
  "gene": "UniProtKB:Q03468",
  "gene_name": "DNA excision repair protein ERCC-6",
  "term_label": "transcription-coupled nucleotide-excision repair"
}